negative regulation of interleukin-24 production [GO:0032708] (biological process) Definition: Any process that stops, prevents, or reduces the frequency, rate, or extent of interleukin-24 production. Relationships: is a type of negative regulation of cytokine production [GO:0001818]; is a type of GO:0032668; negatively regulates interleukin-24 production [GO:0032628] Sources: GOC:mah Also known as: down regulation of interleukin-24 production, down-regulation of interleukin-24 production, downregulation of interleukin-24 production, negative regulation of IL-24 production, inhibition of interleukin-24 production, negative regulation of interleukin-24 biosynthetic process